{
  "term_id": "GO:0043122",
  "gene_name": "C-type lectin domain family 7 member A",
  "gene": "UniProtKB:Q9BXN2",
  "term_label": "regulation of canonical NF-kappaB signal transduction",
  "gene_symbol": "CLEC7A"
}